{
  "gene_name": "Putative uncharacterized protein encoded by LINC00311",
  "term_id": "UNKNOWN:0001",
  "gene_symbol": "LINC00311",
  "gene": "UniProtKB:Q8N616",
  "term_label": "Unknown molecular function"
}